regulation of natural killer cell differentiation [GO:0032823] (biological process) Relationships: is a type of regulation of natural killer cell activation [GO:0032814]; is a type of regulation of lymphocyte differentiation [GO:0045619]; regulates GO:0001779 Note: Note that immunologists typically use the word 'development' to refer to cells of B or T cell lineages undergoing the process that GO describes as 'cell differentiation'. Definition: Any process that modulates the frequency, rate or extent of natural killer cell differentiation. Also known as: regulation of NK cell differentiation, regulation of natural killer cell development Sources: GOC:mah Subtypes: negative regulation of natural killer cell differentiation [GO:0032824], positive regulation of natural killer cell differentiation [GO:0032825], GO:0032826